{
  "gene_name": "Interferon regulatory factor 3",
  "gene_symbol": "IRF3",
  "term_id": "GO:0006357",
  "gene": "UniProtKB:Q14653",
  "term_label": "regulation of transcription by RNA polymerase II"
}